{
  "gene_symbol": "COX5B",
  "term_label": "Unknown molecular function",
  "gene": "UniProtKB:P10606",
  "term_id": "UNKNOWN:0001",
  "gene_name": "Cytochrome c oxidase subunit 5B, mitochondrial"
}